{
  "gene_symbol": "PCSK2",
  "gene_name": "Neuroendocrine convertase 2",
  "term_id": "GO:0016486",
  "term_label": "peptide hormone processing",
  "gene": "UniProtKB:P16519"
}